{
  "term_label": "GTPase activity",
  "gene_symbol": "GPN3",
  "term_id": "GO:0003924",
  "gene_name": "GPN-loop GTPase 3",
  "gene": "UniProtKB:Q9UHW5"
}